{
  "gene_name": "DNA-directed RNA polymerase II subunit RPB2",
  "gene": "UniProtKB:P30876",
  "term_id": "GO:0005665",
  "gene_symbol": "POLR2B",
  "term_label": "RNA polymerase II, core complex"
}